{
  "gene_symbol": "PABPC1L2A",
  "term_label": "Unknown biological process",
  "gene_name": "Polyadenylate-binding protein 1-like 2",
  "term_id": "UNKNOWN:0002",
  "gene": "UniProtKB:Q5JQF8"
}